{
  "gene_symbol": "TDRD5",
  "gene": "UniProtKB:Q8NAT2",
  "term_id": "UNKNOWN:0001",
  "gene_name": "Tudor domain-containing protein 5",
  "term_label": "Unknown molecular function"
}